negative regulation of B cell deletion [GO:0002868] (biological process) Definition: Any process that stops, prevents, or reduces the frequency, rate, or extent of B cell deletion. Also known as: down regulation of B cell deletion, down-regulation of B cell deletion, downregulation of B cell deletion, negative regulation of B lymphocyte deletion, negative regulation of B-cell deletion, negative regulation of B-lymphocyte deletion, inhibition of B cell deletion Sources: GOC:add Subtypes: negative regulation of central B cell deletion [GO:0002899], negative regulation of peripheral B cell deletion [GO:0002909] Relationships: is a type of negative regulation of B cell tolerance induction [GO:0002662]; is a type of GO:0002673; is a type of GO:0002867; is a type of negative regulation of B cell apoptotic process [GO:0002903]; is a type of GO:1904746; negatively regulates GO:0002516